{
  "term_id": "UNKNOWN:0001",
  "gene_name": "Vacuolar protein sorting-associated protein 33B",
  "gene_symbol": "VPS33B",
  "term_label": "Unknown molecular function",
  "gene": "UniProtKB:Q9H267"
}